beta-ureidopropionase activity [GO:0003837] (MF) Definition: Catalysis of the reaction: N-carbamoyl-beta-alanine + H2O = beta-alanine + CO2 + NH3. Relationships: is a type of hydrolase activity, acting on carbon-nitrogen (but not peptide) bonds, in linear amides [GO:0016811] Sources: EC:3.5.1.6 Also known as: N-carbamoyl-beta-alanine amidohydrolase activity